{
  "term_label": "Unknown cellular component",
  "term_id": "UNKNOWN:0003",
  "gene_symbol": "C7orf33",
  "gene_name": "Uncharacterized protein C7orf33",
  "gene": "UniProtKB:Q8WU49"
}